chemokine (C-X-C motif) ligand 13 production [GO:0097391] (biological process) Also known as: CXCL13 production Sources: GOC:rv Relationships: is a type of chemokine production [GO:0032602] Definition: The appearance of chemokine (C-X-C motif) ligand 13 (CXCL13) due to biosynthesis or secretion following a cellular stimulus, resulting in an increase in its intracellular or extracellular levels.